cellular response to raffinose [GO:0097403] (biological process) Definition: Any process that results in a change in state or activity of a cell (in terms of movement, secretion, enzyme production, gene expression, etc.) as a result of a raffinose stimulus. Sources: GOC:al Relationships: is a type of GO:0071322; is a type of response to raffinose [GO:1901545]